{
  "gene": "UniProtKB:Q9H2F5",
  "term_label": "piccolo histone acetyltransferase complex",
  "term_id": "GO:0032777",
  "gene_symbol": "EPC1",
  "gene_name": "Enhancer of polycomb homolog 1"
}